{
  "gene_name": "Receptor-type tyrosine-protein phosphatase R",
  "term_id": "GO:0005886",
  "term_label": "plasma membrane",
  "gene_symbol": "PTPRR",
  "gene": "UniProtKB:Q15256"
}